{
  "gene_symbol": "EIF3H",
  "term_label": "eukaryotic translation initiation factor 3 complex",
  "term_id": "GO:0005852",
  "gene_name": "Eukaryotic translation initiation factor 3 subunit H",
  "gene": "UniProtKB:O15372"
}